{
  "term_id": "GO:0045499",
  "gene_name": "Semaphorin-7A",
  "gene_symbol": "SEMA7A",
  "gene": "UniProtKB:O75326",
  "term_label": "chemorepellent activity"
}